{
  "gene": "UniProtKB:Q9NSI8",
  "term_label": "regulation of intracellular signal transduction",
  "gene_symbol": "SAMSN1",
  "gene_name": "SAM domain-containing protein SAMSN-1",
  "term_id": "GO:1902531"
}